{
  "gene": "UniProtKB:Q2MJR0",
  "term_id": "GO:0019901",
  "term_label": "protein kinase binding",
  "gene_symbol": "SPRED3",
  "gene_name": "Sprouty-related, EVH1 domain-containing protein 3"
}